{
  "gene_symbol": "EPS8L1",
  "term_label": "Rho protein signal transduction",
  "term_id": "GO:0007266",
  "gene_name": "Epidermal growth factor receptor kinase substrate 8-like protein 1",
  "gene": "UniProtKB:Q8TE68"
}